negative regulation of intermediate mesodermal cell fate specification [GO:0048401] (biological process) Definition: Any process that stops, prevents, or reduces the frequency, rate or extent of intermediate mesoderm cell fate specification. Relationships: is_a negative regulation of mesodermal cell fate specification [GO:0042662]; is a type of GO:0048399; negatively regulates intermediate mesodermal cell fate specification [GO:0048398] Sources: GOC:dgh Also known as: down regulation of intermediate mesodermal cell fate specification, down-regulation of intermediate mesodermal cell fate specification, downregulation of intermediate mesodermal cell fate specification, inhibition of intermediate mesodermal cell fate specification